{
  "gene_name": "F-box only protein 38",
  "gene": "UniProtKB:Q6PIJ6",
  "gene_symbol": "FBXO38",
  "term_id": "GO:1990756",
  "term_label": "ubiquitin-like ligase-substrate adaptor activity"
}